pollen maturation [GO:0010152] (biological process) Definition: The final stages of microgametogenesis after the trinucleate stage has been reached resulting in viable pollen grains. Relationships: is a type of developmental maturation [GO:0021700]; BFO_0000050 pollen development [GO:0009555] References: PMID:11595796